{
  "term_label": "ribonucleoprotein complex",
  "gene": "UniProtKB:P17844",
  "gene_name": "Probable ATP-dependent RNA helicase DDX5",
  "gene_symbol": "DDX5",
  "term_id": "GO:1990904"
}